{
  "term_id": "GO:0060090",
  "gene_symbol": "TXNIP",
  "gene": "UniProtKB:Q9H3M7",
  "gene_name": "Thioredoxin-interacting protein",
  "term_label": "molecular adaptor activity"
}